pectoral fin morphogenesis [GO:0035138] (biological process) Relationships: is a type of fin morphogenesis [GO:0033334]; is part of pectoral fin development [GO:0033339] Sources: GOC:dgh Definition: The process in which the anatomical structures of the pectoral fin are generated and organized. Pectoral fins are bilaterally paired fins mounted laterally and located behind the gill covers of fish. These fins are used for lateral mobility and propulsion. Subtypes: embryonic pectoral fin morphogenesis [GO:0035118], post-embryonic pectoral fin morphogenesis [GO:0035130]